cellular response to maltose stimulus [GO:0071328] (biological process) Definition: Any process that results in a change in state or activity of a cell (in terms of movement, secretion, enzyme production, gene expression, etc.) as a result of a maltose stimulus. Sources: GOC:mah Relationships: is a type of response to maltose [GO:0034286]; is a type of cellular response to disaccharide stimulus [GO:0071324]